{
  "term_id": "GO:0006506",
  "term_label": "GPI anchor biosynthetic process",
  "gene": "UniProtKB:Q3MUY2",
  "gene_symbol": "PIGY",
  "gene_name": "Phosphatidylinositol N-acetylglucosaminyltransferase subunit Y"
}